{
  "term_id": "GO:0097484",
  "gene_name": "Transmembrane protein 108",
  "term_label": "dendrite extension",
  "gene_symbol": "TMEM108",
  "gene": "UniProtKB:Q6UXF1"
}